{
  "gene_symbol": "HIRIP3",
  "gene": "UniProtKB:Q9BW71",
  "term_id": "GO:0005634",
  "term_label": "nucleus",
  "gene_name": "HIRA-interacting protein 3"
}